regulation of isotype switching [GO:0045191] (biological process) Subtypes: negative regulation of isotype switching [GO:0045829], GO:0045830, GO:0048293, GO:0048296, GO:0048299, GO:0048302 Relationships: is a type of regulation of DNA recombination [GO:0000018]; is a type of regulation of immunoglobulin production [GO:0002637]; is a type of regulation of immunoglobulin mediated immune response [GO:0002889]; is a type of GO:0050864; regulates GO:0045190 Sources: GOC:ai Definition: Any process that modulates the frequency, rate or extent of isotype switching. Also known as: regulation of class switch recombination, regulation of class switching, regulation of isotype switch recombination